{
  "term_id": "UNKNOWN:0001",
  "gene_name": "Uroplakin-3a",
  "gene": "UniProtKB:O75631",
  "gene_symbol": "UPK3A",
  "term_label": "Unknown molecular function"
}